{
  "term_id": "GO:0071320",
  "gene_symbol": "CRTC1",
  "gene_name": "CREB-regulated transcription coactivator 1",
  "gene": "UniProtKB:Q6UUV9",
  "term_label": "cellular response to cAMP"
}